{
  "gene": "UniProtKB:Q9BXA9",
  "term_id": "GO:0000981",
  "gene_symbol": "SALL3",
  "gene_name": "Sal-like protein 3",
  "term_label": "DNA-binding transcription factor activity, RNA polymerase II-specific"
}